{
  "gene": "UniProtKB:Q5MY95",
  "term_label": "ribonucleoside triphosphate phosphatase activity",
  "gene_name": "Ectonucleoside triphosphate diphosphohydrolase 8",
  "term_id": "GO:0017111",
  "gene_symbol": "ENTPD8"
}